L-alpha-amino acid transmembrane transport [GO:1902475] (biological process) Definition: The directed movement of L-alpha-amino acid across a membrane by means of some agent such as a transporter or a pore. Subtypes: GO:0015813, L-aspartate transmembrane transport [GO:0070778], L-histidine transmembrane transport [GO:0089709], L-tyrosine transmembrane import into vacuole [GO:0090514], L-serine transmembrane import into vacuole [GO:0090516], L-arginine import across plasma membrane [GO:0097638], L-kynurenine transmembrane transport [GO:0140924], L-phenylalanine import across plasma membrane [GO:0140925], GO:1903352, L-lysine transmembrane transport [GO:1903401], GO:1903785, L-leucine import across plasma membrane [GO:1903801], L-glutamine import across plasma membrane [GO:1903803], L-isoleucine import across plasma membrane [GO:1903806], GO:1903807, L-tyrosine import across plasma membrane [GO:1903808], L-asparagine import across plasma membrane [GO:1903811], GO:1903812, GO:1903826, L-proline transmembrane transport [GO:1904555], L-tryptophan transmembrane transport [GO:1904556], L-alanine transmembrane transport [GO:1904557], L-cystine transmembrane transport from lysosomal lumen to cytosol [GO:1904919], L-methionine import across plasma membrane [GO:1905544], L-arginine transmembrane export from vacuole [GO:1990818] Relationships: is a type of amino acid transmembrane transport [GO:0003333]; is_a L-amino acid transport [GO:0015807]; is a type of carboxylic acid transmembrane transport [GO:1905039] References: PMID:14668347 Sources: GOC:TermGenie, GOC:kmv